glutamate secretion [GO:0014047] (biological process) Sources: GOC:ef Definition: The controlled release of glutamate by a cell. The glutamate is the most abundant excitatory neurotransmitter in the nervous system. Subtypes: glutamate secretion, neurotransmission [GO:0061535] Regulation: RO_0002211 by regulation of glutamate secretion [GO:0014048]; RO_0002213 by positive regulation of glutamate secretion [GO:0014049]; negatively regulated by GO:0014050 Relationships: is a type of GO:0006835; is a type of acidic amino acid transport [GO:0015800]; is a type of secretion by cell [GO:0032940]; is a type of nitrogen compound transport [GO:0071705]